cytoplasmic SCF ubiquitin ligase complex [GO:0043223] (cellular component) Relationships: is a type of cytoplasmic ubiquitin ligase complex [GO:0000153]; is a type of SCF ubiquitin ligase complex [GO:0019005] Definition: A ubiquitin ligase complex, located in the cytoplasm, in which a cullin from the Cul1 subfamily and a RING domain protein form the catalytic core; substrate specificity is conferred by a Skp1 adaptor and an F-box protein. SCF complexes are involved in targeting proteins for degradation by the proteasome. The best characterized complexes are those from yeast and mammals (with core subunits named Cdc53/Cul1, Rbx1/Hrt1/Roc1). References: PMID:15571813, PMID:15688063 Also known as: cytoplasmic SCF complex, cytoplasmic Skp1/Cul1/F-box protein complex, cytoplasmic cullin complex